{
  "term_id": "GO:0008013",
  "gene": "UniProtKB:Q8IXH8",
  "gene_name": "Cadherin-like protein 26",
  "gene_symbol": "CDH26",
  "term_label": "beta-catenin binding"
}